L-ornithine import across plasma membrane [GO:0097640] (biological process) Relationships: is a type of amino acid import across plasma membrane [GO:0089718]; is_a GO:1903352 Also known as: L-ornithine import into cell Definition: The directed movement of L-ornithine from outside of a cell, across the plasma membrane and into the cytosol. References: PMID:8195186 Sources: GOC:krc